intracellular transport [GO:0046907] (biological process) Also known as: single organism intracellular transport, single-organism intracellular transport Relationships: is a type of GO:0006810; is a type of GO:0051641; is a type of GO:0051649; occurs in intracellular anatomical structure [GO:0005622] Sources: GOC:ai Definition: The directed movement of substances within a cell. Regulation: RO_0002211 by regulation of intracellular transport [GO:0032386]; negatively regulated by GO:0032387; positively regulated by positive regulation of intracellular transport [GO:0032388] Subtypes: mitochondrial transport [GO:0006839], intracellular protein transport [GO:0006886], endoplasmic reticulum to Golgi vesicle-mediated transport [GO:0006888], vacuolar transport [GO:0007034], nuclear migration [GO:0007097], GO:0015859, synaptic vesicle budding from endosome [GO:0016182], GO:0016197, cytosolic transport [GO:0016482], cytoskeleton-dependent intracellular transport [GO:0030705], intracellular lipid transport [GO:0032365], synaptic vesicle recycling via endosome [GO:0036466], GO:0043485, GO:0043574, cytosol to endoplasmic reticulum transport [GO:0046967], nuclear transport [GO:0051169], Golgi to secretory granule transport [GO:0055107], Golgi to transport vesicle transport [GO:0055108], GO:0090110, receptor-mediated endocytosis involved in cholesterol transport [GO:0090118], cytoplasmic streaming [GO:0099636], clathrin-dependent synaptic vesicle endocytosis [GO:0150007], endoplasmic reticulum to chloroplast transport [GO:1901965], endoplasmic reticulum to cytosol transport [GO:1903513], calcium ion import into sarcoplasmic reticulum [GO:1990036]